{
  "term_label": "nucleoplasm",
  "gene_symbol": "MACROD1",
  "gene": "UniProtKB:Q9BQ69",
  "term_id": "GO:0005654",
  "gene_name": "ADP-ribose glycohydrolase MACROD1"
}